{
  "term_id": "UNKNOWN:0002",
  "gene_name": "Arginine_serine-rich coiled-coil protein 2",
  "term_label": "Unknown biological process",
  "gene_symbol": "RSRC2",
  "gene": "UniProtKB:Q7L4I2"
}